{
  "term_id": "GO:0000389",
  "term_label": "mRNA 3'-splice site recognition",
  "gene_name": "Pre-mRNA-splicing factor ISY1 homolog",
  "gene": "UniProtKB:Q9ULR0",
  "gene_symbol": "ISY1"
}